{
  "gene_symbol": "TMPRSS12",
  "gene_name": "Transmembrane protease serine 12",
  "term_label": "protein processing",
  "gene": "UniProtKB:Q86WS5",
  "term_id": "GO:0016485"
}